Malpighian tubule principal cell differentiation [GO:0061329] (biological process) References: PMID:19783135 Sources: GOC:dph, GOC:mtg_kidney_jan10 Definition: The process in which a relatively unspecialized cell acquires specialized features of a Malpighian tubule principal cell. A Malpighian tubule principal cell is an epithelial secretory cell that transports cations into the lumen of the tubule. Relationships: is a type of epithelial cell differentiation [GO:0030855]; is part of Malpighian tubule development [GO:0072002]